{
  "gene_symbol": "PARD6G",
  "gene_name": "Partitioning defective 6 homolog gamma",
  "term_label": "centrosome cycle",
  "gene": "UniProtKB:Q9BYG4",
  "term_id": "GO:0007098"
}